{
  "gene": "UniProtKB:Q13642",
  "term_label": "Unknown biological process",
  "gene_name": "Four and a half LIM domains protein 1",
  "gene_symbol": "FHL1",
  "term_id": "UNKNOWN:0002"
}